{
  "gene": "UniProtKB:O75496",
  "gene_symbol": "GMNN",
  "term_id": "GO:0045892",
  "term_label": "negative regulation of DNA-templated transcription",
  "gene_name": "Geminin"
}